positive regulation of cortical granule exocytosis by positive regulation of cytosolic calcium ion concentration [GO:0060472] (biological process) Relationships: is a type of positive regulation of calcium ion-dependent exocytosis [GO:0045956]; is a type of regulation of cell activation [GO:0050865]; is a type of GO:0060470; is a type of GO:2000243; positively regulates cortical granule exocytosis [GO:0060471] Definition: Any process that activates or increases the frequency, rate or extent of cortical granule exocytosis by directing movement of calcium ions (Ca2+) into the cytosol. Also known as: positive regulation of cortical granule exocytosis by elevation of cytosolic calcium ion concentration Sources: GOC:dph